thiosulfate-thiol sulfurtransferase activity [GO:0050337] (molecular function) Definition: Catalysis of the reaction: thiosulfate + 2 glutathione = glutathione disulfide + hydrogen sulfide + sulfite + 2 H+. Relationships: is a type of sulfurtransferase activity [GO:0016783] Sources: RHEA:14505 Also known as: thiosulphate-thiol sulphurtransferase activity, glutathione-dependent thiosulfate reductase activity, sulfane reductase activity, sulfane sulfurtransferase activity, thiosulfate:thiol sulfurtransferase activity